nitrate reductase [NAD(P)H] activity [GO:0050463] (molecular function) Definition: Catalysis of the reaction: nitrite + NAD(P)+ + H2O = nitrate + NAD(P)H + H+. Sources: EC:1.7.1.2 Also known as: NAD(P)H bispecific nitrate reductase activity, NAD(P)H-nitrate reductase activity, NAD(P)H2:nitrate oxidoreductase activity, NAD(P)H:nitrate oxidoreductase activity, assimilatory NAD(P)H-nitrate reductase activity, assimilatory nitrate reductase activity, nitrate reductase (reduced nicotinamide adenine dinucleotide (phosphate)) activity, nitrate reductase NAD(P)H activity, nitrate reductase [NAD(P)H2], nitrite:NAD(P)+ oxidoreductase activity Relationships: is a type of nitrate reductase activity [GO:0008940]; is a type of oxidoreductase activity, acting on other nitrogenous compounds as donors, with NAD or NADP as acceptor [GO:0046857] Subtypes: GO:0009703, GO:0050464